{
  "term_label": "Unknown molecular function",
  "gene_name": "CD177 antigen",
  "gene_symbol": "CD177",
  "gene": "UniProtKB:Q8N6Q3",
  "term_id": "UNKNOWN:0001"
}